negative regulation of myeloid cell differentiation [GO:0045638] (biological process) Also known as: down regulation of myeloid cell differentiation, down-regulation of myeloid cell differentiation, downregulation of myeloid cell differentiation, inhibition of myeloid cell differentiation Subtypes: GO:0002762, negative regulation of erythrocyte differentiation [GO:0045647], negative regulation of megakaryocyte differentiation [GO:0045653], GO:1905220 Sources: GOC:go_curators Definition: Any process that stops, prevents, or reduces the frequency, rate or extent of myeloid cell differentiation. Relationships: is a type of negative regulation of cell differentiation [GO:0045596]; is a type of GO:0045637; negatively regulates GO:0030099